{
  "term_label": "mitochondrial intermembrane space",
  "gene": "UniProtKB:O43715",
  "gene_symbol": "TRIAP1",
  "term_id": "GO:0005758",
  "gene_name": "TP53-regulated inhibitor of apoptosis 1"
}